{
  "term_label": "cytoplasm",
  "term_id": "GO:0005737",
  "gene": "UniProtKB:Q96DH6",
  "gene_name": "RNA-binding protein Musashi homolog 2",
  "gene_symbol": "MSI2"
}